{
  "gene": "UniProtKB:Q16620",
  "gene_symbol": "NTRK2",
  "term_id": "GO:0043679",
  "gene_name": "BDNF_NT-3 growth factors receptor",
  "term_label": "axon terminus"
}